{
  "gene_symbol": "KRTAP3-1",
  "term_id": "UNKNOWN:0001",
  "gene_name": "Keratin-associated protein 3-1",
  "gene": "UniProtKB:Q9BYR8",
  "term_label": "Unknown molecular function"
}